{
  "gene_symbol": "GAS2L2",
  "gene": "UniProtKB:Q8NHY3",
  "gene_name": "GAS2-like protein 2",
  "term_label": "cytoplasm",
  "term_id": "GO:0005737"
}